2'-deoxyguanosine DNA ADP-ribosyltransferase activity [GO:0030591] (molecular function) Also known as: NAD DNA ADP-ribosyltransferase activity Definition: Catalysis of the transfer of the ADP-ribose group of NAD+ to the amino group at N2 of 2'-deoxyguanosine to yield N2-(alpha-ADP-ribos-1-yl)-2'-deoxyguanosine and its beta form. Relationships: is a type of NAD DNA ADP-ribosyltransferase activity [GO:0140294] References: PMID:11592983